negative regulation of cellular process [GO:0048523] (biological process) Subtypes: negative regulation of cilium movement [GO:0003354], GO:0007162, negative regulation of cell population proliferation [GO:0008285], negative regulation of metabolic process [GO:0009892], negative regulation of cellular response to nitrogen starvation [GO:0010516], negative regulation of cell communication [GO:0010648], negative regulation of lipid storage [GO:0010888], GO:0030308, negative regulation of cell killing [GO:0031342], negative regulation of myelination [GO:0031642], negative regulation of intracellular transport [GO:0032387], GO:0034763, negative regulation of programmed cell death [GO:0043069], negative regulation of cell differentiation [GO:0045596], negative regulation of cell cycle [GO:0045786], negative regulation of establishment of competence for transformation [GO:0045808], negative regulation of cytolysis [GO:0045918], negative regulation of cell activation [GO:0050866], negative regulation of cellular component organization [GO:0051129], GO:0051283, negative regulation of cell division [GO:0051782], negative regulation of cell adhesion molecule production [GO:0060354], negative regulation of hepatic stellate cell contraction [GO:0061875], negative regulation of plus-end directed microtubule sliding [GO:0062168], negative regulation of ribosome biogenesis [GO:0090071], negative regulation of protein targeting to membrane [GO:0090315], GO:0106021, negative regulation of cardiac muscle cell contraction [GO:0106135], GO:0110014, negative regulation of cellular response to phosphate starvation [GO:0140256], negative regulation of pre-B cell receptor expression [GO:0140646], negative regulation of cellular response to heat [GO:1900035], negative regulation of cellular response to hypoxia [GO:1900038], GO:1900068, negative regulation of cellular hyperosmotic salinity response [GO:1900070], negative regulation of cellular response to insulin stimulus [GO:1900077], negative regulation of single-species biofilm formation [GO:1900191], negative regulation of phenotypic switching [GO:1900240], negative regulation of cellular response to oxidative stress [GO:1900408], negative regulation of cellular response to caffeine [GO:1901181], GO:1901967, negative regulation of stomatal opening [GO:1902457], GO:1902804, GO:1902873, negative regulation of melanosome transport [GO:1902909], GO:1903333, negative regulation of cell wall organization or biogenesis [GO:1903339], GO:1903531, GO:1903573, negative regulation of cellular response to amino acid starvation [GO:1903574], GO:1903919, negative regulation of muscle filament sliding [GO:1904113], GO:1904299, negative regulation of myofibroblast contraction [GO:1904329], negative regulation of spore germination [GO:1904360], negative regulation of establishment of bipolar cell polarity [GO:1904846], GO:1904932, negative regulation of vascular associated smooth muscle cell dedifferentiation [GO:1905175], negative regulation of protein localization to membrane [GO:1905476], negative regulation of cellular response to manganese ion [GO:1905803], negative regulation of cellular response to gamma radiation [GO:1905844], negative regulation of cellular response to oxidopamine [GO:1905847], GO:1905888, negative regulation of cellular response to alcohol [GO:1905958], GO:2000146, negative regulation of ribonucleoprotein complex localization [GO:2000198], negative regulation of binding of sperm to zona pellucida [GO:2000360], negative regulation of cellular response to testosterone stimulus [GO:2000655], negative regulation of cellular response to X-ray [GO:2000684], negative regulation of dense core granule biogenesis [GO:2000706], negative regulation of establishment or maintenance of cell polarity regulating cell shape [GO:2000770], negative regulation of cellular senescence [GO:2000773], negative regulation of cellular response to drug [GO:2001039], negative regulation of septum digestion after cytokinesis [GO:2001042] Sources: GOC:jid Definition: Any process that stops, prevents, or reduces the frequency, rate or extent of a cellular process, any of those that are carried out at the cellular level, but are not necessarily restricted to a single cell. For example, cell communication occurs among more than one cell, but occurs at the cellular level. Relationships: is a type of GO:0048519; is a type of regulation of cellular process [GO:0050794]; negatively regulates cellular process [GO:0009987] Also known as: down regulation of cellular process, down-regulation of cellular process, downregulation of cellular process, negative regulation of cellular physiological process, inhibition of cellular process